{
  "gene_name": "ATP-binding cassette sub-family D member 3",
  "term_label": "ATP binding",
  "gene_symbol": "ABCD3",
  "gene": "UniProtKB:P28288",
  "term_id": "GO:0005524"
}